{
  "term_label": "non-canonical Wnt signaling pathway",
  "gene": "UniProtKB:Q9NPG1",
  "gene_name": "Frizzled-3",
  "gene_symbol": "FZD3",
  "term_id": "GO:0035567"
}